positive regulation of ureteric bud formation [GO:0072107] (biological process) Definition: Any process that increases the rate or extent of the developmental process pertaining to the initial formation of the ureteric bud from the Wolffian duct. Sources: GOC:mtg_kidney_jan10 Relationships: is a type of regulation of ureteric bud formation [GO:0072106]; is a type of positive regulation of animal organ morphogenesis [GO:0110110]; is a type of positive regulation of epithelial tube formation [GO:1905278]; positively regulates GO:0060676